{
  "gene": "UniProtKB:Q9BXJ4",
  "term_id": "GO:0099550",
  "gene_name": "Complement C1q tumor necrosis factor-related protein 3",
  "gene_symbol": "C1QTNF3",
  "term_label": "trans-synaptic signaling, modulating synaptic transmission"
}